positive regulation of protein targeting to vacuolar membrane [GO:1900485] (biological process) Definition: Any process that activates or increases the frequency, rate or extent of protein targeting to vacuolar membrane. Sources: GOC:TermGenie Also known as: up regulation of protein targeting to vacuolar membrane, up-regulation of protein targeting to vacuolar membrane, upregulation of protein targeting to vacuolar membrane, activation of protein targeting to vacuolar membrane Relationships: is a type of positive regulation of protein targeting to membrane [GO:0090314]; is_a positive regulation of intracellular protein transport [GO:0090316]; is a type of regulation of protein targeting to vacuolar membrane [GO:1900483]; is a type of GO:1903337; is a type of GO:1905477; positively regulates GO:0044395